{
  "gene_symbol": "POLI",
  "gene": "UniProtKB:Q9UNA4",
  "term_id": "GO:0003887",
  "gene_name": "DNA polymerase iota",
  "term_label": "DNA-directed DNA polymerase activity"
}